protein farnesyltransferase complex [GO:0005965] (cellular component) Sources: GOC:mah Relationships: is a type of GO:1990234; is part of GO:0005737 Definition: A protein complex that possesses protein farnesyltransferase activity.